{
  "term_label": "apical plasma membrane",
  "gene": "UniProtKB:P41440",
  "gene_name": "Reduced folate transporter",
  "term_id": "GO:0016324",
  "gene_symbol": "SLC19A1"
}